{
  "term_id": "GO:0006790",
  "gene_symbol": "CHST3",
  "term_label": "sulfur compound metabolic process",
  "gene": "UniProtKB:Q7LGC8",
  "gene_name": "Carbohydrate sulfotransferase 3"
}